SREBP-SCAP complex retention in endoplasmic reticulum [GO:0036316] (biological process) References: PMID:16525117 Sources: GOC:bf Definition: Any process in which the SREBP-SCAP complex is maintained in the endoplasmic reticulum and prevented from moving elsewhere. The SREBP-SCAP complex is formed by the association of sterol regulatory element binding protein (SREBP) and SREBP-cleavage-activating protein (SCAP). In the absence of sterols, the SREBP-SCAP complex is packaged into COPII vesicles and travels to the Golgi apparatus to be processed. In the presence of sterols, the complex binds ER-resident proteins such as INSIG, which retain the complex in the ER. Relationships: is a type of GO:0035437; is a type of negative regulation of SREBP signaling pathway [GO:2000639]; is part of cellular response to sterol [GO:0036315] Note: Consider also annotating to the cellular component term: SREBP-SCAP-Insig complex ; GO:0032937.